{
  "term_id": "UNKNOWN:0003",
  "gene": "UniProtKB:Q9NQ79",
  "gene_name": "Cartilage acidic protein 1",
  "gene_symbol": "CRTAC1",
  "term_label": "Unknown cellular component"
}